{
  "gene": "UniProtKB:P02647",
  "gene_name": "Apolipoprotein A-I",
  "gene_symbol": "APOA1",
  "term_id": "GO:0042627",
  "term_label": "chylomicron"
}